{
  "term_id": "GO:0042391",
  "gene": "UniProtKB:P36544",
  "gene_name": "Neuronal acetylcholine receptor subunit alpha-7",
  "gene_symbol": "CHRNA7",
  "term_label": "regulation of membrane potential"
}